{
  "term_id": "GO:0009898",
  "gene_symbol": "RGS2",
  "term_label": "cytoplasmic side of plasma membrane",
  "gene_name": "Regulator of G-protein signaling 2",
  "gene": "UniProtKB:P41220"
}